{
  "gene": "UniProtKB:Q9UI47",
  "gene_symbol": "CTNNA3",
  "term_label": "adherens junction",
  "gene_name": "Catenin alpha-3",
  "term_id": "GO:0005912"
}